{
  "gene_name": "Apoptosis-stimulating of p53 protein 1",
  "term_id": "GO:0002039",
  "gene_symbol": "PPP1R13B",
  "gene": "UniProtKB:Q96KQ4",
  "term_label": "p53 binding"
}